{
  "gene_symbol": "RHOXF1",
  "gene": "UniProtKB:Q8NHV9",
  "term_label": "regulation of transcription by RNA polymerase II",
  "term_id": "GO:0006357",
  "gene_name": "Rhox homeobox family member 1"
}